{
  "term_label": "Unknown biological process",
  "term_id": "UNKNOWN:0002",
  "gene_symbol": "SMIM10",
  "gene_name": "Small integral membrane protein 10",
  "gene": "UniProtKB:Q96HG1"
}